negative regulation of antibacterial peptide production [GO:0002787] (BP) Subtypes: GO:0002798, GO:0002809 Sources: GOC:add Also known as: down regulation of antibacterial peptide production, down-regulation of antibacterial peptide production, downregulation of antibacterial peptide production, inhibition of antibacterial peptide production Relationships: is a type of negative regulation of antimicrobial peptide production [GO:0002785]; is a type of GO:0002786; is a type of negative regulation of defense response to bacterium [GO:1900425]; negatively regulates antibacterial peptide production [GO:0002778] Definition: Any process that stops, prevents, or reduces the frequency, rate, or extent of antibacterial peptide production.